{
  "term_id": "GO:0061627",
  "term_label": "S-methylmethionine-homocysteine S-methyltransferase activity",
  "gene_name": "S-methylmethionine--homocysteine S-methyltransferase BHMT2",
  "gene_symbol": "BHMT2",
  "gene": "UniProtKB:Q9H2M3"
}